{
  "term_id": "GO:0002020",
  "gene_symbol": "PZP",
  "term_label": "protease binding",
  "gene": "UniProtKB:P20742",
  "gene_name": "Pregnancy zone protein"
}